{
  "gene_name": "Metalloreductase STEAP3",
  "term_id": "GO:0052851",
  "term_label": "ferric-chelate reductase (NADPH) activity",
  "gene": "UniProtKB:Q658P3",
  "gene_symbol": "STEAP3"
}